{
  "gene_name": "Olfactory receptor 2G6",
  "term_id": "GO:0004984",
  "gene_symbol": "OR2G6",
  "gene": "UniProtKB:Q5TZ20",
  "term_label": "olfactory receptor activity"
}